GDP-L-fucose synthase activity [GO:0050577] (molecular function) Also known as: GDP-4-keto-6-deoxy-D-mannose-3,5-epimerase-4-reductase activity, GDP-L-fucose:NADP+ 4-oxidoreductase (3,5-epimerizing), GDP-fucose synthetase activity Definition: Catalysis of the reaction: GDP-L-fucose + NAD+ = GDP-4-dehydro-6-deoxy-D-mannose + NADH + H+. Relationships: is_a oxidoreductase activity, acting on the CH-OH group of donors, NAD or NADP as acceptor [GO:0016616]; is part of GDP-L-fucose biosynthetic process [GO:0042350] Sources: EC:1.1.1.271, MetaCyc:1.1.1.271-RXN